{
  "gene": "UniProtKB:Q9Y333",
  "gene_name": "U6 snRNA-associated Sm-like protein LSm2",
  "term_id": "GO:0003723",
  "gene_symbol": "LSM2",
  "term_label": "RNA binding"
}